dorsal/ventral axon guidance [GO:0033563] (biological process) Also known as: dorsal-ventral axon guidance, dorsal/ventral axon pathfinding, dorsoventral axon guidance Sources: GOC:dph, GOC:kmv, GOC:tb Relationships: is a type of GO:0007411 Regulation: regulated by regulation of dorsal/ventral axon guidance [GO:1905815]; RO_0002212 by negative regulation of dorsal/ventral axon guidance [GO:1905816]; positively regulated by positive regulation of dorsal/ventral axon guidance [GO:1905817] Definition: The process in which the migration of an axon growth cone is directed to a specific target site along the dorsal-ventral body axis in response to a combination of attractive and repulsive cues. The dorsal/ventral axis is defined by a line that runs orthogonal to both the anterior/posterior and left/right axes. The dorsal end is defined by the upper or back side of an organism. The ventral end is defined by the lower or front side of an organism.